{
  "gene": "UniProtKB:Q6IF63",
  "term_id": "GO:0005886",
  "gene_symbol": "OR52W1",
  "gene_name": "Olfactory receptor 52W1",
  "term_label": "plasma membrane"
}